long-chain fatty-acyl-glutamate deacylase activity [GO:0008421] (molecular function) Relationships: is a type of hydrolase activity, acting on carbon-nitrogen (but not peptide) bonds, in linear amides [GO:0016811] Definition: Catalysis of the reaction: N-long-chain-fatty-acyl-L-glutamate + H2O = a fatty acid anion + L-glutamate. Also known as: long-chain fatty acyl-glutamate deacylase activity, long-chain-fatty-acyl-glutamate deacylase activity, N-long-chain-fatty-acyl-L-glutamate amidohydrolase activity, long-chain acylglutamate amidase activity, long-chain aminoacylase activity Sources: EC:3.5.1.55